nucleoside oxidase (hydrogen peroxide-forming) activity [GO:0033716] (molecular function) Definition: Catalysis of the reactions: adenosine + 2 O2 = 9-riburonosyladenine + 2 hydrogen peroxide. Relationships: is a type of oxidoreductase activity, acting on the CH-OH group of donors, oxygen as acceptor [GO:0016899] Note: Two other reactions might be associated with this activity: (1a) adenosine + O2 = 5'-dehydroadenosine + hydrogen peroxide, and (1b) 5'-dehydroadenosine + O2 = 9-riburonosyladenine + hydrogen peroxide. Sources: EC:1.1.3.39, RHEA:15489 Also known as: nucleoside:oxygen 5'-oxidoreductase (hydrogen peroxide-forming) activity